{
  "term_id": "UNKNOWN:0002",
  "term_label": "Unknown biological process",
  "gene": "UniProtKB:Q6UXB8",
  "gene_symbol": "PI16",
  "gene_name": "Peptidase inhibitor 16"
}